{
  "gene": "UniProtKB:O75943",
  "gene_symbol": "RAD17",
  "term_label": "chromatin-protein adaptor activity",
  "gene_name": "Cell cycle checkpoint protein RAD17",
  "term_id": "GO:0140463"
}